{
  "gene": "UniProtKB:Q07283",
  "term_label": "protein-macromolecule adaptor activity",
  "gene_name": "Trichohyalin",
  "gene_symbol": "TCHH",
  "term_id": "GO:0030674"
}